{
  "gene_symbol": "KAZALD1",
  "gene": "UniProtKB:Q96I82",
  "term_id": "GO:0048018",
  "gene_name": "Kazal-type serine protease inhibitor domain-containing protein 1",
  "term_label": "receptor ligand activity"
}